{
  "gene": "UniProtKB:Q9P273",
  "gene_symbol": "TENM3",
  "gene_name": "Teneurin-3",
  "term_id": "GO:0046982",
  "term_label": "protein heterodimerization activity"
}